{
  "term_id": "GO:0003950",
  "gene_symbol": "PARP6",
  "gene_name": "Protein mono-ADP-ribosyltransferase PARP6",
  "term_label": "NAD+ poly-ADP-ribosyltransferase activity",
  "gene": "UniProtKB:Q2NL67"
}